positive regulation of tetrapyrrole biosynthetic process from glycine and succinyl-CoA [GO:1901415] (biological process) Definition: Any process that activates or increases the frequency, rate or extent of tetrapyrrole biosynthetic process from glycine and succinyl-CoA. Also known as: activation of tetrapyrrole anabolism from glycine and succinyl-CoA, activation of tetrapyrrole biosynthesis from glycine and succinyl-CoA, activation of tetrapyrrole formation from glycine and succinyl-CoA, activation of tetrapyrrole synthesis from glycine and succinyl-CoA, positive regulation of tetrapyrrole anabolism from glycine and succinyl-CoA, positive regulation of tetrapyrrole biosynthesis from glycine and succinyl-CoA, positive regulation of tetrapyrrole formation from glycine and succinyl-CoA, positive regulation of tetrapyrrole synthesis from glycine and succinyl-CoA, up regulation of tetrapyrrole anabolism from glycine and succinyl-CoA, up regulation of tetrapyrrole biosynthesis from glycine and succinyl-CoA, up regulation of tetrapyrrole biosynthetic process from glycine and succinyl-CoA, up regulation of tetrapyrrole formation from glycine and succinyl-CoA, up regulation of tetrapyrrole synthesis from glycine and succinyl-CoA, up-regulation of tetrapyrrole anabolism from glycine and succinyl-CoA, up-regulation of tetrapyrrole biosynthesis from glycine and succinyl-CoA, up-regulation of tetrapyrrole biosynthetic process from glycine and succinyl-CoA, up-regulation of tetrapyrrole formation from glycine and succinyl-CoA, up-regulation of tetrapyrrole synthesis from glycine and succinyl-CoA, upregulation of tetrapyrrole anabolism from glycine and succinyl-CoA, upregulation of tetrapyrrole biosynthesis from glycine and succinyl-CoA, upregulation of tetrapyrrole biosynthetic process from glycine and succinyl-CoA, upregulation of tetrapyrrole formation from glycine and succinyl-CoA, upregulation of tetrapyrrole synthesis from glycine and succinyl-CoA, activation of tetrapyrrole biosynthetic process from glycine and succinyl-CoA Relationships: is a type of positive regulation of amide metabolic process [GO:0034250]; is a type of GO:0045764; is a type of positive regulation of phosphate metabolic process [GO:0045937]; is_a positive regulation of small molecule metabolic process [GO:0062013]; is a type of regulation of tetrapyrrole biosynthetic process from glycine and succinyl-CoA [GO:1901413]; is a type of positive regulation of tetrapyrrole biosynthetic process [GO:1901465]; positively regulates tetrapyrrole biosynthetic process from glycine and succinyl-CoA [GO:0033527] Sources: GOC:TermGenie, GOC:mengo_curators